lifelong otolith mineralization [GO:0031174] (BP) Definition: The formation and growth of otoliths throughout the life of the organism. Otoliths are the large extracellular ear-stones of the fish inner ear, produced by precipitation of specific crystal forms of calcium carbonate on organic matrices. The otolith enlarges throughout the life of the fish, as layers of calcium carbonate are added. References: PMID:15581873 Sources: GOC:dsf Relationships: is a type of otolith mineralization [GO:0045299]